{
  "term_label": "Unknown biological process",
  "gene": "UniProtKB:Q53RY4",
  "gene_symbol": "KRTCAP3",
  "term_id": "UNKNOWN:0002",
  "gene_name": "Keratinocyte-associated protein 3"
}